{
  "gene_name": "CLIP-associating protein 1",
  "term_label": "spindle microtubule",
  "term_id": "GO:0005876",
  "gene_symbol": "CLASP1",
  "gene": "UniProtKB:Q7Z460"
}